{
  "gene_symbol": "CCL4",
  "term_label": "positive regulation of cell migration",
  "gene": "UniProtKB:P13236",
  "gene_name": "C-C motif chemokine 4",
  "term_id": "GO:0030335"
}